{
  "gene_symbol": "UBE3A",
  "gene_name": "Ubiquitin-protein ligase E3A",
  "term_id": "GO:0005829",
  "gene": "UniProtKB:Q05086",
  "term_label": "cytosol"
}